tRNA adenosine deamination to inosine [GO:0140023] (biological process) Relationships: is a type of tRNA modification [GO:0006400] Also known as: A-to-I tRNA editing Definition: The removal of an amine group from an adenosine to produce inosine within a tRNA molecule. References: PMID:27974624